{
  "term_id": "GO:0005634",
  "gene": "UniProtKB:P0DI82",
  "gene_symbol": "TRAPPC2B",
  "gene_name": "Trafficking protein particle complex subunit 2B",
  "term_label": "nucleus"
}